regulation of lung ciliated cell differentiation [GO:1901246] (BP) Sources: GOC:BHF, GOC:TermGenie Relationships: is a type of regulation of epithelial cell differentiation [GO:0030856]; regulates lung ciliated cell differentiation [GO:0061141] Definition: Any process that modulates the frequency, rate or extent of lung ciliated cell differentiation. Subtypes: negative regulation of lung ciliated cell differentiation [GO:1901247], positive regulation of lung ciliated cell differentiation [GO:1901248]